{
  "term_label": "GTPase activity",
  "gene": "UniProtKB:O43236",
  "term_id": "GO:0003924",
  "gene_name": "Septin-4",
  "gene_symbol": "SEPTIN4"
}